{
  "term_id": "GO:0072534",
  "gene": "UniProtKB:O14594",
  "gene_name": "Neurocan core protein",
  "term_label": "perineuronal net",
  "gene_symbol": "NCAN"
}